{
  "gene_name": "Immunoglobulin lambda variable 3-22",
  "gene_symbol": "IGLV3-22",
  "gene": "UniProtKB:A0A075B6J6",
  "term_id": "UNKNOWN:0001",
  "term_label": "Unknown molecular function"
}